{
  "gene_symbol": "SHROOM4",
  "gene_name": "Protein Shroom4",
  "gene": "UniProtKB:Q9ULL8",
  "term_label": "apical plasma membrane",
  "term_id": "GO:0016324"
}